{
  "term_label": "protein-N-terminal-glutamate acetyltransferase activity",
  "gene_symbol": "NAA11",
  "term_id": "GO:1990190",
  "gene_name": "N-alpha-acetyltransferase 11",
  "gene": "UniProtKB:Q9BSU3"
}